{
  "gene": "UniProtKB:Q9UBU6",
  "gene_symbol": "FAM8A1",
  "term_id": "UNKNOWN:0001",
  "term_label": "Unknown molecular function",
  "gene_name": "Protein FAM8A1"
}